{
  "term_label": "regulation of transcription by RNA polymerase II",
  "term_id": "GO:0006357",
  "gene": "UniProtKB:O95238",
  "gene_name": "SAM pointed domain-containing Ets transcription factor",
  "gene_symbol": "SPDEF"
}